indole-3-glycerol-phosphate synthase activity [GO:0004425] (molecular function) Definition: Catalysis of the reaction: 1-(2-carboxyphenylamino)-1-deoxy-D-ribulose 5-phosphate = 1-(indol-3-yl)glycerol 3-phosphate + CO2 + H2O. Sources: EC:4.1.1.48 Relationships: is a type of carboxy-lyase activity [GO:0016831] Also known as: 1-(2-carboxyphenylamino)-1-deoxy-D-ribulose-5-phosphate carboxy-lyase (cyclizing), 1-(2-carboxyphenylamino)-1-deoxy-D-ribulose-5-phosphate carboxy-lyase [cyclizing; 1-C-(3-indolyl)-glycerol-3-phosphate-forming], indole-3-glycerophosphate synthase activity, indoleglycerol phosphate synthase activity, indoleglycerol phosphate synthetase activity